{
  "term_label": "homophilic cell-cell adhesion",
  "gene_name": "Cell adhesion molecule 3",
  "gene_symbol": "CADM3",
  "gene": "UniProtKB:Q8N126",
  "term_id": "GO:0007156"
}